{
  "gene": "UniProtKB:O43566",
  "term_id": "GO:0005634",
  "gene_name": "Regulator of G-protein signaling 14",
  "term_label": "nucleus",
  "gene_symbol": "RGS14"
}